de novo centriole assembly involved in multi-ciliated epithelial cell differentiation [GO:0098535] (BP) References: PMID:24075808, PMID:5111878, PMID:5661997 Sources: GOC:cilia, GOC:dos Note: In most eukaryotic cells, 'centriole' (GO:0005814) and 'ciliary basal body' (GO:0036064) represent a common entity that cycles through its function in cell division, then ciliogenesis, then cell division again. However, these structures are modified extensively as they transition into each other, and may contain different proteins, specific to each component. Also known as: de novo centriole assembly, de novo centriole assembly via deuterosome, centriole amplification, deuterosomal basal body biogenesis, deuterosome pathway, deuterosome-mediated centriole biogenesis, multiciliation, multiciliogenesis Definition: Centriole assembly in which a centriole arises de novo by a process involving an electron-dense structure known as a deuterosome, rather than by duplication of an existing centriole, and occurring as part of multi-ciliated epithelial cell differentiation. Relationships: is a type of de novo centriole assembly [GO:0097742]; is part of multi-ciliated epithelial cell differentiation [GO:1903251]